{
  "gene_symbol": "CRABP2",
  "gene": "UniProtKB:P29373",
  "term_label": "nucleus",
  "gene_name": "Cellular retinoic acid-binding protein 2",
  "term_id": "GO:0005634"
}